{
  "term_label": "regulation of cytokine production",
  "gene_symbol": "ZBTB37",
  "gene": "UniProtKB:Q5TC79",
  "gene_name": "Zinc finger and BTB domain-containing protein 37",
  "term_id": "GO:0001817"
}